beta-hydroxybutyrate transmembrane transporter activity [GO:0097253] (molecular function) Definition: Enables the transfer of beta-hydroxybutyrate from one side of a membrane to the other. Beta-hydroxybutyrate is the conjugate base of (R)-3-hydroxybutyric acid. References: PMID:22302940 Sources: GOC:dsf Also known as: (R)-3-hydroxybutyrate transmembrane transporter activity, 3-hydroxybutanoic acid transmembrane transporter activity Relationships: is_a GO:0015245; is a type of GO:0015665